{
  "gene_symbol": "BBS2",
  "gene_name": "Bardet-Biedl syndrome 2 protein",
  "term_label": "Unknown molecular function",
  "term_id": "UNKNOWN:0001",
  "gene": "UniProtKB:Q9BXC9"
}